{
  "term_id": "GO:0061630",
  "gene_name": "Tripartite motif-containing protein 44",
  "gene": "UniProtKB:Q96DX7",
  "gene_symbol": "TRIM44",
  "term_label": "ubiquitin protein ligase activity"
}